{
  "gene": "UniProtKB:Q15695",
  "term_id": "GO:0089701",
  "term_label": "U2AF complex",
  "gene_name": "Putative U2 small nuclear ribonucleoprotein auxiliary factor 35 kDa subunit-related protein 1",
  "gene_symbol": "ZRSR2P1"
}